{
  "term_id": "GO:0006644",
  "gene": "UniProtKB:Q6T4P5",
  "gene_name": "Phospholipid phosphatase-related protein type 3",
  "gene_symbol": "PLPPR3",
  "term_label": "phospholipid metabolic process"
}